{
  "term_label": "delta DNA polymerase complex",
  "gene_symbol": "POLD3",
  "gene": "UniProtKB:Q15054",
  "gene_name": "DNA polymerase delta subunit 3",
  "term_id": "GO:0043625"
}